regulation of plasminogen activation [GO:0010755] (biological process) Definition: Any process that modulates the rate, frequency or extent of plasminogen activation. Plasminogen activation is the process in which plasminogen is processed to plasmin. Sources: GOC:BHF, GOC:dph, GOC:tb Relationships: is a type of GO:0070613; regulates GO:0031639 Subtypes: GO:0010756, negative regulation of plasminogen activation [GO:0010757]